oligodendrocyte progenitor proliferation [GO:0070444] (biological process) References: PMID:15504915 Sources: GOC:mah, GOC:sl Relationships: is a type of GO:0061351; is part of gliogenesis [GO:0042063] Also known as: oligodendrocyte precursor proliferation Regulation: RO_0002211 by regulation of oligodendrocyte progenitor proliferation [GO:0070445]; negatively regulated by negative regulation of oligodendrocyte progenitor proliferation [GO:0070446]; positively regulated by GO:0070447 Definition: The multiplication or reproduction of oligodendrocyte progenitor cells by cell division, resulting in the expansion of their population. Oligodendrocyte progenitors give rise to oligodendrocytes, which form the insulating myelin sheath of axons in the central nervous system.